response to antineoplastic agent [GO:0097327] (biological process) Definition: Any process that results in a change in state or activity of a cell or an organism (in terms of movement, secretion, enzyme production, gene expression, etc.) as a result of an antineoplastic agent stimulus. An antineoplastic agent is a substance that inhibits or prevents the proliferation of neoplasms. Sources: GOC:pr Relationships: is a type of GO:0042221